{
  "gene_name": "Rho guanine nucleotide exchange factor 5",
  "gene": "UniProtKB:Q12774",
  "term_label": "regulation of actin cytoskeleton organization",
  "gene_symbol": "ARHGEF5",
  "term_id": "GO:0032956"
}